{
  "term_id": "GO:0034063",
  "term_label": "stress granule assembly",
  "gene": "UniProtKB:Q8ND56",
  "gene_symbol": "LSM14A",
  "gene_name": "Protein LSM14 homolog A"
}